{
  "gene": "UniProtKB:Q01113",
  "gene_name": "Interleukin-9 receptor",
  "gene_symbol": "IL9R",
  "term_id": "GO:0004919",
  "term_label": "interleukin-9 receptor activity"
}